{
  "gene_name": "Tyrosine-protein phosphatase non-receptor type 21",
  "term_label": "protein tyrosine phosphatase activity",
  "term_id": "GO:0004725",
  "gene": "UniProtKB:Q16825",
  "gene_symbol": "PTPN21"
}